coenzyme A catabolic process [GO:0015938] (biological process) Definition: The chemical reactions and pathways resulting in the breakdown of coenzyme A, 3'-phosphoadenosine-(5')diphospho(4')pantatheine, an acyl carrier in many acylation and acyl-transfer reactions in which the intermediate is a thiol ester. Sources: ISBN:0198547684 Also known as: CoA catabolism, coenzyme A breakdown, coenzyme A catabolism, coenzyme A degradation Relationships: is a type of GO:0015936; is a type of sulfur compound catabolic process [GO:0044273]; is a type of GO:0072523; is a type of nucleoside phosphate catabolic process [GO:1901292]